{
  "gene_symbol": "CSGALNACT2",
  "gene_name": "Chondroitin sulfate N-acetylgalactosaminyltransferase 2",
  "term_label": "chondroitin sulfate proteoglycan biosynthetic process",
  "gene": "UniProtKB:Q8N6G5",
  "term_id": "GO:0050650"
}